actinorhodin catabolic process [GO:1901111] (biological process) Definition: The chemical reactions and pathways resulting in the breakdown of actinorhodin. Sources: GOC:TermGenie, GOC:yaf, UniPathway:UPA00173 Relationships: is a type of dicarboxylic acid catabolic process [GO:0043649] Also known as: actinorhodin breakdown, actinorhodin catabolism, actinorhodin degradation